{
  "gene_name": "Spectrin alpha chain, erythrocytic 1",
  "gene": "UniProtKB:P02549",
  "term_label": "actin filament binding",
  "term_id": "GO:0051015",
  "gene_symbol": "SPTA1"
}